UBR1-RAD6 ubiquitin ligase complex [GO:1990303] (cellular component) Relationships: is a type of intracellular protein-containing complex [GO:0140535]; is a type of transferase complex [GO:1990234] Definition: A ubiquitin ligase complex consisting of UBR1 and RAD6 components. It polyubiquitinates proteins containing non-acetylated N-terminal residues causing their subsequent degradation by the proteasome as part of the Ac/N-End Rule pathway. It recognizes non-acetylated N-terminal methionine if it is followed by a hydrophobic residue. Additionally, it acts in an N-end rule independent manner as a component of a novel quality control pathway for proteins synthesized on cytosolic ribosomes. Note: This complex has been identified in Saccharomyces cerevisiae (P19812) - see PMID:19531475 (inferred from direct assay). References: PMID:19531475 Sources: GOC:bhm Also known as: UBR1-RAD6 complex